L-glutamate import involved in cellular response to nitrogen starvation [GO:1901481] (biological process) Also known as: L-glutamate uptake involved in cellular response to nitrogen starvation Definition: Any L-glutamate import that is involved in cellular response to nitrogen starvation. Relationships: is a type of GO:0051938; is part of GO:0006995 Sources: GOC:TermGenie